{
  "term_id": "GO:0003700",
  "term_label": "DNA-binding transcription factor activity",
  "gene": "UniProtKB:Q66K89",
  "gene_symbol": "E4F1",
  "gene_name": "Transcription factor E4F1"
}